{
  "term_label": "dynactin binding",
  "gene_symbol": "SNX6",
  "term_id": "GO:0034452",
  "gene_name": "Sorting nexin-6",
  "gene": "UniProtKB:Q9UNH7"
}